[acyl-carrier-protein] phosphodiesterase activity [GO:0008770] (molecular function) Sources: EC:3.1.4.14 Definition: Catalysis of the reaction: [acyl-carrier protein] + H2O = 4'-phosphopantetheine + apoprotein. Relationships: is a type of phosphoric diester hydrolase activity [GO:0008081]; is a type of catalytic activity, acting on a protein [GO:0140096] Also known as: ACP phosphodiesterase activity, [acyl-carrier protein] phosphodiesterase activity, ACP hydrolyase activity, AcpH, [acyl-carrier-protein] 4'-pantetheine-phosphohydrolase activity, acyl-carrier-protein 4'-pantetheine-phosphohydrolase activity, acyl-carrier-protein phosphodiesterase activity, holo-acyl-carrier-protein 4'-pantetheine-phosphohydrolase activity